{
  "term_id": "GO:0005886",
  "gene": "UniProtKB:P00450",
  "term_label": "plasma membrane",
  "gene_name": "Ceruloplasmin",
  "gene_symbol": "CP"
}